{
  "term_label": "RNA polymerase II cis-regulatory region sequence-specific DNA binding",
  "gene_name": "Homeobox protein NANOGP8",
  "term_id": "GO:0000978",
  "gene_symbol": "NANOGP8",
  "gene": "UniProtKB:Q6NSW7"
}